{
  "term_label": "plasma membrane",
  "gene_symbol": "PCDHGA8",
  "term_id": "GO:0005886",
  "gene": "UniProtKB:Q9Y5G5",
  "gene_name": "Protocadherin gamma-A8"
}